{
  "term_id": "GO:0045892",
  "term_label": "negative regulation of DNA-templated transcription",
  "gene": "UniProtKB:Q96EB6",
  "gene_symbol": "SIRT1",
  "gene_name": "NAD-dependent protein deacetylase sirtuin-1"
}